{
  "gene": "UniProtKB:Q0VDE8",
  "gene_name": "Adipogenin",
  "term_id": "GO:0050873",
  "term_label": "brown fat cell differentiation",
  "gene_symbol": "ADIG"
}